succinate-CoA ligase complex (GDP-forming) [GO:0045244] (cellular component) Definition: A heterodimeric enzyme complex, usually composed of an alpha and beta chain. Functions in the TCA cycle, hydrolyzing succinyl-CoA into succinate and CoA, thereby forming GTP. Also known as: succinyl-CoA synthetase, GDP-forming References: PMID:27487822 Sources: GOC:jl Relationships: is a type of succinate-CoA ligase complex [GO:0042709]